{
  "gene_name": "Acyl-coenzyme A diphosphatase NUDT19",
  "gene_symbol": "NUDT19",
  "gene": "UniProtKB:A8MXV4",
  "term_id": "UNKNOWN:0002",
  "term_label": "Unknown biological process"
}